{
  "term_id": "GO:0035556",
  "gene_name": "Pro-neuregulin-1, membrane-bound isoform",
  "gene_symbol": "NRG1",
  "term_label": "intracellular signal transduction",
  "gene": "UniProtKB:Q02297"
}